mesenchymal cell condensation involved in mammary fat development [GO:0060647] (biological process) References: PMID:12558599 Sources: GOC:dph Relationships: is a type of cell-cell adhesion [GO:0098609]; is part of mammary gland fat development [GO:0060611] Definition: The cell adhesion process in which mammary mesenchyme cells adhere to one another in the initial stages of the formation of mammary fat development.